{
  "term_label": "amphisome",
  "term_id": "GO:0044753",
  "gene_symbol": "SQSTM1",
  "gene_name": "Sequestosome-1",
  "gene": "UniProtKB:Q13501"
}